{
  "gene": "UniProtKB:P02655",
  "gene_name": "Apolipoprotein C-II",
  "gene_symbol": "APOC2",
  "term_id": "GO:0034363",
  "term_label": "intermediate-density lipoprotein particle"
}